{
  "term_label": "nucleus",
  "gene_symbol": "CDYL",
  "term_id": "GO:0005634",
  "gene": "UniProtKB:Q9Y232",
  "gene_name": "Chromodomain Y-like protein"
}